insect visual primordium development [GO:0001748] (biological process) Relationships: is a type of anatomical structure development [GO:0048856] Definition: The process whose specific outcome is the progression of the optic placode over time, from its formation to the mature structure. During embryonic stage 12 the placode starts to invaginate, forming a pouch. Cells that will form Bolwig's organ segregate from the ventral lip of this pouch, remaining in the head epidermis. The remainder of the invagination loses contact with the outer surface and becomes the optic lobe. An example of this process is found in Drosophila melanogaster. References: PMID:8402833 Sources: GOC:mtg_sensu Also known as: optic placode development, optic lobe and Bolwig's organ precursor development, optic lobe placode development